{
  "gene_symbol": "CFC1B",
  "gene": "UniProtKB:P0CG36",
  "term_label": "anterior/posterior pattern specification",
  "term_id": "GO:0009952",
  "gene_name": "Cryptic family protein 1B"
}